{
  "gene_name": "Ribonuclease P protein subunit p38",
  "term_label": "ribonuclease P activity",
  "gene": "UniProtKB:P78345",
  "gene_symbol": "RPP38",
  "term_id": "GO:0004526"
}